{
  "gene": "UniProtKB:Q9BT56",
  "gene_symbol": "SPX",
  "term_label": "positive regulation of gastro-intestinal system smooth muscle contraction",
  "term_id": "GO:1904306",
  "gene_name": "Spexin"
}